positive regulation of metaphase/anaphase transition of meiosis II [GO:1905191] (biological process) Definition: Any process that activates or increases the frequency, rate or extent of metaphase/anaphase transition of meiosis II. Relationships: is_a positive regulation of metaphase/anaphase transition of meiotic cell cycle [GO:1902104]; is a type of regulation of metaphase/anaphase transition of meiosis II [GO:1905189]; positively regulates metaphase/anaphase transition of meiosis II [GO:1990950] References: PMID:21389117 Sources: GOC:TermGenie, GO_REF:0000058 Also known as: positive regulation of meiosis II metaphase/anaphase transition